{
  "term_label": "RNA polymerase II cis-regulatory region sequence-specific DNA binding",
  "gene": "UniProtKB:Q9Y2Y4",
  "gene_name": "Zinc finger and BTB domain-containing protein 32",
  "gene_symbol": "ZBTB32",
  "term_id": "GO:0000978"
}